{
  "gene_name": "Zinc finger and BTB domain-containing protein 37",
  "gene_symbol": "ZBTB37",
  "term_label": "DNA-binding transcription repressor activity, RNA polymerase II-specific",
  "term_id": "GO:0001227",
  "gene": "UniProtKB:Q5TC79"
}